caveolin-mediated endocytosis of virus by host cell [GO:0075513] (biological process) Also known as: viral entry into host cell via caveolae-mediated endocytosis, viral penetration via caveolae-mediated endocytosis followed by endosome disruption, viral entry into host cell via caveolin-mediated endocytosis Relationships: is a type of receptor-mediated endocytosis of virus by host cell [GO:0019065]; is a type of caveolin-mediated endocytosis [GO:0072584] Definition: Any caveolin-mediated endocytosis that is involved in the uptake of a virus into a host cell. Begins when material is taken up into plasma membrane caveolae - specialized lipid rafts that form 50-70 nm flask-shaped invaginations of the plasma membrane - which then pinch off to form endocytic caveolar carriers containing the virus. Sources: GOC:bf, GOC:jl, VZ:976